{
  "term_label": "regulation of DNA-templated transcription",
  "gene_name": "Zinc finger and BTB domain-containing protein 11",
  "term_id": "GO:0006355",
  "gene": "UniProtKB:O95625",
  "gene_symbol": "ZBTB11"
}